{
  "gene_symbol": "ESR2",
  "gene": "UniProtKB:Q92731",
  "gene_name": "Estrogen receptor beta",
  "term_id": "GO:0006357",
  "term_label": "regulation of transcription by RNA polymerase II"
}